myosin VI binding [GO:0070853] (MF) Definition: Binding to a class VI myosin. The myosin VI heavy chain has a single IQ motif in the neck and a tail region with a coiled coil domain followed by a unique globular domain, a unique insertion that enables myosin VI to move towards the pointed or minus end of actin filaments. References: PMID:15473855 Sources: GOC:mah Relationships: is a type of myosin binding [GO:0017022] Subtypes: myosin VI heavy chain binding [GO:0070854], myosin VI light chain binding [GO:0070856]